{
  "gene_name": "Phosphoribosyl pyrophosphate synthase-associated protein 2",
  "gene": "UniProtKB:O60256",
  "term_id": "GO:0030234",
  "gene_symbol": "PRPSAP2",
  "term_label": "enzyme regulator activity"
}